{
  "term_id": "GO:0005737",
  "gene_name": "Acetyl-coenzyme A synthetase, cytoplasmic",
  "term_label": "cytoplasm",
  "gene": "UniProtKB:Q9NR19",
  "gene_symbol": "ACSS2"
}